{
  "term_label": "actin filament binding",
  "gene_name": "Transmembrane protein 201",
  "gene_symbol": "TMEM201",
  "term_id": "GO:0051015",
  "gene": "UniProtKB:Q5SNT2"
}